uracil phosphoribosyltransferase activity [GO:0004845] (molecular function) Definition: Catalysis of the reaction: diphosphate + UMP = 5-phospho-alpha-D-ribose 1-diphosphate + uracil. Also known as: UMP diphosphorylase activity, UMP pyrophosphorylase activity, UMP:diphosphate phospho-alpha-D-ribosyltransferase activity, UMP:pyrophosphate phosphoribosyltransferase activity, UPRTase activity, uridine 5'-phosphate pyrophosphorylase activity, uridine monophosphate pyrophosphorylase activity, uridylate pyrophosphorylase activity, uridylic pyrophosphorylase activity Relationships: is a type of GO:0016763 Sources: EC:2.4.2.9, RHEA:13017